{
  "gene": "UniProtKB:P35670",
  "gene_name": "Copper-transporting ATPase 2",
  "term_id": "GO:0006878",
  "gene_symbol": "ATP7B",
  "term_label": "intracellular copper ion homeostasis"
}